neuronal stem cell population maintenance [GO:0097150] (biological process) Relationships: is a type of GO:0019827 References: PMID:11399758 Sources: CL:0000047, GOC:dos, GOC:yaf Definition: Any process in by an organism or tissue maintains a population of neuronal stem cells.